{
  "term_id": "GO:1904292",
  "gene": "UniProtKB:Q15011",
  "gene_name": "Homocysteine-responsive endoplasmic reticulum-resident ubiquitin-like domain member 1 protein",
  "gene_symbol": "HERPUD1",
  "term_label": "regulation of ERAD pathway"
}